{
  "term_id": "GO:0051899",
  "gene_name": "Neuronal acetylcholine receptor subunit alpha-2",
  "gene": "UniProtKB:Q15822",
  "term_label": "membrane depolarization",
  "gene_symbol": "CHRNA2"
}